{
  "gene": "UniProtKB:P00739",
  "term_label": "zymogen activation",
  "gene_symbol": "HPR",
  "term_id": "GO:0031638",
  "gene_name": "Haptoglobin-related protein"
}